{
  "term_label": "Unknown cellular component",
  "gene_symbol": "IRX2-DT",
  "gene": "UniProtKB:Q86SI9",
  "term_id": "UNKNOWN:0003",
  "gene_name": "Putative uncharacterized protein IRX2-DT"
}